{
  "gene_symbol": "CASTOR1",
  "term_label": "arginine binding",
  "gene": "UniProtKB:Q8WTX7",
  "gene_name": "Cytosolic arginine sensor for mTORC1 subunit 1",
  "term_id": "GO:0034618"
}